{
  "gene_name": "Inositol 1,4,5-trisphosphate receptor type 2",
  "term_id": "GO:0016529",
  "term_label": "sarcoplasmic reticulum",
  "gene_symbol": "ITPR2",
  "gene": "UniProtKB:Q14571"
}